photosynthesis, light harvesting [GO:0009765] (biological process) Definition: Absorption and transfer of the energy absorbed from light photons between photosystem reaction centers. Sources: GOC:sm Also known as: energy dissipation Relationships: is a type of generation of precursor metabolites and energy [GO:0006091]; BFO_0000050 photosynthesis, light reaction [GO:0019684] Subtypes: GO:0009768, photosynthesis, light harvesting in photosystem II [GO:0009769]